positive regulation of Golgi to plasma membrane protein transport [GO:0042998] (biological process) Definition: Any process that activates or increases the frequency, rate or extent of the transport of proteins from the Golgi to the plasma membrane. Also known as: up regulation of Golgi to plasma membrane protein transport, up-regulation of Golgi to plasma membrane protein transport, upregulation of Golgi to plasma membrane protein transport, activation of Golgi to plasma membrane protein transport, stimulation of Golgi to plasma membrane protein transport Relationships: is a type of GO:0042996; is a type of positive regulation of protein transport [GO:0051222]; is a type of positive regulation of protein localization to plasma membrane [GO:1903078]; positively regulates Golgi to plasma membrane protein transport [GO:0043001] Sources: GOC:jl